cellular response to 1-aminocyclopropane-1-carboxylic acid [GO:0071213] (biological process) Sources: GOC:mah Relationships: is a type of GO:0009961; is a type of cellular response to amino acid stimulus [GO:0071230]; is a type of cellular response to nitrogen compound [GO:1901699]; is a type of GO:1901701 Definition: Any process that results in a change in state or activity of a cell (in terms of movement, secretion, enzyme production, gene expression, etc.) as a result of a 1-aminocyclopropane-1-carboxylic acid stimulus.